{
  "term_id": "UNKNOWN:0002",
  "gene_name": "Galectin-7",
  "gene": "UniProtKB:P47929",
  "gene_symbol": "LGALS7",
  "term_label": "Unknown biological process"
}